{
  "term_id": "UNKNOWN:0002",
  "gene_name": "Monoacylglycerol_Diacylglycerol O-acyltransferase",
  "gene_symbol": "TMEM68",
  "term_label": "Unknown biological process",
  "gene": "UniProtKB:Q96MH6"
}